{
  "term_id": "GO:0005737",
  "gene_symbol": "DUSP10",
  "gene_name": "Dual specificity protein phosphatase 10",
  "term_label": "cytoplasm",
  "gene": "UniProtKB:Q9Y6W6"
}